{
  "gene": "UniProtKB:Q08AG7",
  "term_label": "spindle",
  "term_id": "GO:0005819",
  "gene_symbol": "MZT1",
  "gene_name": "Mitotic-spindle organizing protein 1"
}